{
  "term_id": "GO:0005819",
  "term_label": "spindle",
  "gene": "UniProtKB:Q8N0Z3",
  "gene_symbol": "SPICE1",
  "gene_name": "Spindle and centriole-associated protein 1"
}